protein ADP-ribosyltransferase-substrate adaptor activity [GO:0140768] (molecular function) Definition: An enzyme-substrate adaptor that bings together a protein ADP-ribosyl transferase and its substrate. Relationships: is a type of enzyme-substrate adaptor activity [GO:0140767] References: PMID:32028527